{
  "term_id": "GO:0140311",
  "gene": "UniProtKB:O14604",
  "gene_name": "Thymosin beta-4, Y-chromosomal",
  "term_label": "protein sequestering activity",
  "gene_symbol": "TMSB4Y"
}